caffeoyl-CoA: alcohol caffeoyl transferase activity [GO:0090430] (molecular function) Sources: GOC:pz Definition: Catalysis of the reaction: caffeoyl-CoA + a saturated primary alcohol = an alkyl caffeate + CoA. Relationships: is a type of acyltransferase activity, transferring groups other than amino-acyl groups [GO:0016747]